{
  "term_label": "plasma membrane",
  "gene": "UniProtKB:P43630",
  "gene_name": "Killer cell immunoglobulin-like receptor 3DL2",
  "gene_symbol": "KIR3DL2",
  "term_id": "GO:0005886"
}